ureteric bud development [GO:0001657] (biological process) Sources: GOC:go_curators Relationships: is a type of mesonephric tubule development [GO:0072164] Definition: The process whose specific outcome is the progression of the ureteric bud over time, from its formation to the mature structure.